{
  "term_id": "GO:0030991",
  "term_label": "intraciliary transport particle A",
  "gene_name": "Intraflagellar transport protein 122 homolog",
  "gene_symbol": "IFT122",
  "gene": "UniProtKB:Q9HBG6"
}